{
  "gene_name": "Rhophilin-2",
  "gene": "UniProtKB:Q8IUC4",
  "term_id": "UNKNOWN:0003",
  "gene_symbol": "RHPN2",
  "term_label": "Unknown cellular component"
}